{
  "gene_name": "ALK tyrosine kinase receptor",
  "term_label": "transmembrane receptor protein tyrosine kinase activity",
  "term_id": "GO:0004714",
  "gene_symbol": "ALK",
  "gene": "UniProtKB:Q9UM73"
}